{
  "gene_name": "Transcription factor SOX-30",
  "term_label": "DNA-binding transcription factor activity, RNA polymerase II-specific",
  "term_id": "GO:0000981",
  "gene": "UniProtKB:O94993",
  "gene_symbol": "SOX30"
}